{
  "gene": "UniProtKB:Q8IZU8",
  "term_label": "dermatan sulfate proteoglycan metabolic process",
  "term_id": "GO:0050655",
  "gene_name": "Dermatan-sulfate epimerase-like protein",
  "gene_symbol": "DSEL"
}